{
  "gene_symbol": "CUEDC1",
  "term_id": "UNKNOWN:0002",
  "term_label": "Unknown biological process",
  "gene": "UniProtKB:Q9NWM3",
  "gene_name": "CUE domain-containing protein 1"
}